{
  "gene": "UniProtKB:P11686",
  "term_id": "UNKNOWN:0002",
  "term_label": "Unknown biological process",
  "gene_name": "Pulmonary surfactant-associated protein C",
  "gene_symbol": "SFTPC"
}